{
  "gene_name": "Thioredoxin domain-containing protein 9",
  "gene": "UniProtKB:O14530",
  "term_id": "UNKNOWN:0001",
  "gene_symbol": "TXNDC9",
  "term_label": "Unknown molecular function"
}